{
  "gene_symbol": "GGT5",
  "gene_name": "Glutathione hydrolase 5 proenzyme",
  "term_id": "GO:1901750",
  "gene": "UniProtKB:P36269",
  "term_label": "leukotriene D4 biosynthetic process"
}